cellodextrin metabolic process [GO:2000889] (biological process) Definition: The chemical reactions and pathways involving a cellodextrin. Also known as: cellodextrin metabolism Relationships: is a type of oligosaccharide metabolic process [GO:0009311]; is a type of glucan metabolic process [GO:0044042] Subtypes: cellodextrin catabolic process [GO:2000890] Sources: GOC:obol